{
  "gene": "UniProtKB:Q8WUQ7",
  "gene_name": "Splicing factor Cactin",
  "gene_symbol": "CACTIN",
  "term_label": "spliceosomal complex",
  "term_id": "GO:0005681"
}